{
  "term_id": "GO:0003729",
  "gene_name": "Zinc finger CCCH domain-containing protein 11C",
  "term_label": "mRNA binding",
  "gene": "UniProtKB:P0DQW0",
  "gene_symbol": "ZC3H11C"
}